{
  "gene": "UniProtKB:Q969Q1",
  "gene_name": "E3 ubiquitin-protein ligase TRIM63",
  "term_id": "GO:0045087",
  "gene_symbol": "TRIM63",
  "term_label": "innate immune response"
}